{
  "gene_name": "E3 ubiquitin-protein ligase MYCBP2",
  "term_id": "GO:0005886",
  "term_label": "plasma membrane",
  "gene": "UniProtKB:O75592",
  "gene_symbol": "MYCBP2"
}